Ral protein signal transduction [GO:0032484] (biological process) Relationships: is_a small GTPase-mediated signal transduction [GO:0007264] Definition: An intracellular signaling cassette in which a small monomeric GTPase of the RaI subfamily relays a signal. Regulation: RO_0002211 by regulation of Ral protein signal transduction [GO:0032485] Sources: GOC:mah